pathogen-containing vacuole lumen [GO:0140222] (cellular component) Also known as: lumen of a pathogen-containing vacuole, pathogen-containing compartment lumen, pathogen-containing vacuolar lumen, pathogen inclusion lumen Definition: The enclosed volume within the sealed membrane of a pathogen-containing vacuole. References: PMID:10560000, PMID:26842840 Relationships: is a type of membrane-enclosed lumen [GO:0031974]; BFO_0000050 pathogen-containing vacuole [GO:0140220]